{
  "gene": "UniProtKB:O00744",
  "gene_symbol": "WNT10B",
  "gene_name": "Protein Wnt-10b",
  "term_label": "neuron differentiation",
  "term_id": "GO:0030182"
}